aromatic amino acid:proton symporter activity [GO:0015494] (molecular function) Definition: Enables the transfer of a solute or solutes from one side of a membrane to the other according to the reaction: aromatic amino acid(out) + H+(out) = aromatic amino acid(in) + H+(in). Also known as: aromatic amino acid:hydrogen symporter activity Subtypes: phenylalanine:proton symporter activity [GO:0015492] Sources: TC:2.A.3.1.3 Relationships: is a type of aromatic amino acid transmembrane transporter activity [GO:0015173]; is a type of solute:proton symporter activity [GO:0015295]